apoptotic process involved in salivary gland cavitation [GO:0060663] (biological process) Also known as: apoptosis involved in salivary gland cavitation Relationships: is a type of GO:0060609; is part of salivary gland cavitation [GO:0060662] References: PMID:17336109 Sources: GOC:dph, GOC:mtg_apoptosis Definition: Any apoptotic process in which the solid core of the gland is hollowed out to form the duct.